{
  "term_label": "Unknown molecular function",
  "gene_symbol": "FAHD2B",
  "term_id": "UNKNOWN:0001",
  "gene_name": "Fumarylacetoacetate hydrolase domain-containing protein 2B",
  "gene": "UniProtKB:Q6P2I3"
}